{
  "term_label": "arachidonate metabolic process",
  "gene_name": "Polyunsaturated fatty acid lipoxygenase ALOX12",
  "term_id": "GO:0019369",
  "gene_symbol": "ALOX12",
  "gene": "UniProtKB:P18054"
}